{
  "gene": "UniProtKB:P26951",
  "gene_name": "Interleukin-3 receptor subunit alpha",
  "term_id": "GO:0019221",
  "term_label": "cytokine-mediated signaling pathway",
  "gene_symbol": "IL3RA"
}